{
  "gene_name": "Interferon-inducible double-stranded RNA-dependent protein kinase activator A",
  "term_label": "siRNA processing",
  "gene": "UniProtKB:O75569",
  "term_id": "GO:0030422",
  "gene_symbol": "PRKRA"
}